{
  "term_id": "GO:0007165",
  "gene_symbol": "CSNK1G2",
  "gene_name": "Casein kinase I isoform gamma-2",
  "gene": "UniProtKB:P78368",
  "term_label": "signal transduction"
}